{
  "gene": "UniProtKB:P0DMV9",
  "gene_symbol": "HSPA1B",
  "term_id": "GO:0042026",
  "term_label": "protein refolding",
  "gene_name": "Heat shock 70 kDa protein 1B"
}